juvenile hormone mediated signaling pathway [GO:0035626] (biological process) References: PMID:28285758, PMID:29888456 Definition: The series of molecular signals initiated by a juvenile hormone binding to its receptor, a bHLH-PAS transcription factor, to regulate gene expression. Also known as: juvenile hormone mediated signalling pathway, juvenile hormone-mediated signaling pathway Relationships: is a type of hormone-mediated signaling pathway [GO:0009755]; is a type of intracellular receptor signaling pathway [GO:0030522]